{
  "gene_name": "Ig-like domain-containing protein (Fragment)",
  "gene": "UniProtKB:A0A0G2JRQ6",
  "gene_symbol": "A0A0G2JRQ6",
  "term_label": "immune response",
  "term_id": "GO:0006955"
}